{
  "term_id": "GO:0005886",
  "term_label": "plasma membrane",
  "gene_name": "Plexin-D1",
  "gene": "UniProtKB:Q9Y4D7",
  "gene_symbol": "PLXND1"
}